{
  "gene_symbol": "CABIN1",
  "term_id": "GO:0003714",
  "term_label": "transcription corepressor activity",
  "gene": "UniProtKB:Q9Y6J0",
  "gene_name": "Calcineurin-binding protein cabin-1"
}